{
  "term_label": "lamellipodium",
  "term_id": "GO:0030027",
  "gene_symbol": "PDPN",
  "gene": "UniProtKB:Q86YL7",
  "gene_name": "Podoplanin"
}